{
  "gene_symbol": "STAT2",
  "gene_name": "Signal transducer and activator of transcription 2",
  "gene": "UniProtKB:P52630",
  "term_id": "GO:0000978",
  "term_label": "RNA polymerase II cis-regulatory region sequence-specific DNA binding"
}